{
  "gene": "UniProtKB:Q9NX94",
  "gene_symbol": "WBP1L",
  "gene_name": "WW domain binding protein 1-like",
  "term_id": "UNKNOWN:0003",
  "term_label": "Unknown cellular component"
}